copper ion import across prospore membrane [GO:0097430] (biological process) Also known as: copper ion import into ascospore-type prospore, copper ion transport into forespores Relationships: is a type of copper ion transmembrane transport [GO:0035434] Definition: The directed movement of copper ions from outside of a cell, across an ascospore-type prospore membrane and into the cytosol. References: PMID:21828039 Sources: GOC:al, GOC:vw